{
  "term_label": "regulation of transcription by RNA polymerase II",
  "gene_name": "Transcription factor Sp2",
  "term_id": "GO:0006357",
  "gene": "UniProtKB:Q02086",
  "gene_symbol": "SP2"
}